{
  "gene_name": "Iron-responsive element-binding protein 2",
  "term_id": "GO:0003994",
  "term_label": "aconitate hydratase activity",
  "gene": "UniProtKB:P48200",
  "gene_symbol": "IREB2"
}